gamma-aminobutyric acid reuptake [GO:0051936] (biological process) Relationships: is a type of GO:0015812; is a type of amino acid neurotransmitter reuptake [GO:0051933] Definition: The uptake of gamma-aminobutyric acid (GABA, 4-aminobutyrate) by neurons or glial cells. This process leads to inactivation and recycling of neurotransmitters. Sources: ISBN:0123668387 Also known as: GABA recycling, gamma-aminobutyric acid recycling, GABA reuptake, gamma-aminobutyric acid uptake involved in synaptic transmission, GABA import into glial cell, GABA import into neuron, gamma-aminobutyric acid import into glial cell, gamma-aminobutyric acid import into neuron, gamma-aminobutyric acid uptake during transmission of nerve impulse Regulation: regulated by regulation of gamma-aminobutyric acid uptake involved in transmission of nerve impulse [GO:0051947]; negatively regulated by negative regulation of gamma-aminobutyric acid uptake involved in transmission of nerve impulse [GO:0051949]; positively regulated by positive regulation of gamma-aminobutyric acid uptake involved in transmission of nerve impulse [GO:0051950]